{
  "term_id": "UNKNOWN:0001",
  "gene_symbol": "BAIAP2L2",
  "term_label": "Unknown molecular function",
  "gene_name": "Brain-specific angiogenesis inhibitor 1-associated protein 2-like protein 2",
  "gene": "UniProtKB:Q6UXY1"
}